{
  "gene_name": "ER membrane protein complex subunit 6",
  "gene_symbol": "EMC6",
  "gene": "UniProtKB:Q9BV81",
  "term_id": "UNKNOWN:0001",
  "term_label": "Unknown molecular function"
}